{
  "term_label": "nucleus",
  "gene_symbol": "ETS2",
  "gene_name": "Protein C-ets-2",
  "term_id": "GO:0005634",
  "gene": "UniProtKB:P15036"
}